{
  "gene_name": "C-C chemokine receptor type 4",
  "gene": "UniProtKB:P51679",
  "gene_symbol": "CCR4",
  "term_label": "C-C chemokine receptor activity",
  "term_id": "GO:0016493"
}